{
  "term_id": "UNKNOWN:0001",
  "gene_symbol": "CHCHD1",
  "term_label": "Unknown molecular function",
  "gene_name": "Small ribosomal subunit protein mS37",
  "gene": "UniProtKB:Q96BP2"
}